regulation of chaperone-mediated autophagy [GO:1904714] (biological process) Definition: Any process that modulates the frequency, rate or extent of chaperone-mediated autophagy. References: PMID:20176123 Sources: GOC:PARL, GOC:TermGenie, GOC:pad, GO_REF:0000058 Also known as: regulation of CMA Relationships: is a type of regulation of autophagy [GO:0010506]; is a type of GO:0042176; RO_0002211 chaperone-mediated autophagy [GO:0061684] Subtypes: negative regulation of chaperone-mediated autophagy [GO:1904715], positive regulation of chaperone-mediated autophagy [GO:1904716]